{
  "term_label": "extracellular space",
  "gene": "UniProtKB:Q08397",
  "gene_symbol": "LOXL1",
  "gene_name": "Lysyl oxidase homolog 1",
  "term_id": "GO:0005615"
}